maturation of LSU-rRNA from tricistronic rRNA transcript (SSU-rRNA, 5.8S rRNA, LSU-rRNA) [GO:0000463] (biological process) Relationships: is a type of maturation of LSU-rRNA [GO:0000470] Sources: GOC:curators Definition: Any process involved in the maturation of a precursor Large SubUnit (LSU) ribosomal RNA (rRNA) molecule into a mature LSU-rRNA molecule from the pre-rRNA molecule originally produced as a tricistronic rRNA transcript that contains the Small Subunit (SSU) rRNA, 5.8S rRNA, and Large Subunit (LSU) in that order from 5' to 3' along the primary transcript.